{
  "gene": "UniProtKB:A6NH57",
  "gene_name": "Putative ADP-ribosylation factor-like protein 5C",
  "term_id": "GO:1903292",
  "gene_symbol": "ARL5C",
  "term_label": "protein localization to Golgi membrane"
}